{
  "gene_name": "Membrane metallo-endopeptidase-like 1",
  "term_label": "plasma membrane",
  "gene": "UniProtKB:Q495T6",
  "term_id": "GO:0005886",
  "gene_symbol": "MMEL1"
}